{
  "gene_symbol": "RNF222",
  "term_id": "UNKNOWN:0002",
  "term_label": "Unknown biological process",
  "gene_name": "RING finger protein 222",
  "gene": "UniProtKB:A6NCQ9"
}